{
  "gene_symbol": "UBL5",
  "gene": "UniProtKB:Q9BZL1",
  "term_id": "GO:0000398",
  "gene_name": "Ubiquitin-like protein 5",
  "term_label": "mRNA splicing, via spliceosome"
}